{
  "gene_symbol": "KCTD5",
  "gene": "UniProtKB:Q9NXV2",
  "term_id": "GO:0031463",
  "gene_name": "BTB_POZ domain-containing protein KCTD5",
  "term_label": "Cul3-RING ubiquitin ligase complex"
}